{
  "term_label": "sodium:phosphate symporter activity",
  "term_id": "GO:0005436",
  "gene_symbol": "SLC34A3",
  "gene": "UniProtKB:Q8N130",
  "gene_name": "Sodium-dependent phosphate transport protein 2C"
}